positive regulation of protein metabolic process [GO:0051247] (biological process) Relationships: is a type of positive regulation of macromolecule metabolic process [GO:0010604]; is a type of regulation of protein metabolic process [GO:0051246]; positively regulates protein metabolic process [GO:0019538] Sources: GOC:ai Definition: Any process that activates or increases the frequency, rate or extent of the chemical reactions and pathways involving a protein. Also known as: positive regulation of cellular protein metabolic process, positive regulation of cellular protein metabolism, positive regulation of protein metabolism, up regulation of cellular protein metabolic process, up regulation of protein metabolic process, up-regulation of cellular protein metabolic process, up-regulation of protein metabolic process, upregulation of cellular protein metabolic process, upregulation of protein metabolic process, activation of cellular protein metabolic process, activation of protein metabolic process, stimulation of cellular protein metabolic process, stimulation of protein metabolic process Subtypes: positive regulation of protein modification process [GO:0031401], GO:0032725, positive regulation of hepatocyte growth factor production [GO:0032726], positive regulation of lymphotoxin A production [GO:0032761], positive regulation of translation [GO:0045727], positive regulation of protein catabolic process [GO:0045732], positive regulation of proteolysis [GO:0045862], GO:0046985, positive regulation of lipoprotein metabolic process [GO:0050747], positive regulation of amyloid precursor protein catabolic process [GO:1902993], GO:1903020, GO:1903319, positive regulation of amyloid fibril formation [GO:1905908]